lumenal side of membrane [GO:0098576] (cellular component) Definition: Any side (leaflet) of a membrane that faces the lumen of an organelle. Relationships: is a type of GO:0098552 Sources: GOC:dos Subtypes: GO:0098538, GO:0098547, lumenal side of endoplasmic reticulum membrane [GO:0098553], lumenal side of endosome membrane [GO:0098565], lumenal side of lysosomal membrane [GO:0098575], matrix side of mitochondrial inner membrane [GO:0099617], lumenal side of cis-Golgi network membrane [GO:0140178], lumenal side of cis-Golgi cisternae membrane [GO:0160277], lumenal side of medial-Golgi cisterna membrane [GO:0160280], lumenal side of trans-Golgi network membrane [GO:0160282], lumenal side of trans-Golgi cisternae membrane [GO:0160289]